{
  "term_label": "mitochondrion",
  "gene_symbol": "BAD",
  "gene": "UniProtKB:Q92934",
  "gene_name": "Bcl2-associated agonist of cell death",
  "term_id": "GO:0005739"
}